2,7,4'-trihydroxyisoflavanone-4'-O-methyltransferase activity [GO:0102670] (MF) Definition: Catalysis of the reaction: 2,4',7-trihydroxyisoflavanone + S-adenosyl-L-methionine = H+ + 2,7-dihydroxy-4'-methoxyisoflavanone + S-adenosyl-L-homocysteine. Sources: EC:2.1.1.212, GOC:pz Relationships: is a type of methyltransferase activity [GO:0008168]